inositol-1,3,4-trisphosphate 5-kinase activity [GO:0052726] (molecular function) Also known as: 1D-myo-inositol-trisphosphate 5-kinase activity, IP3 5-kinase activity, inositol-trisphosphate 5-kinase activity, inositol 1,3,4-trisphosphate 5-kinase activity, ins(1,3,4)P(3) 5-kinase activity Relationships: is a type of inositol trisphosphate kinase activity [GO:0051766] Definition: Catalysis of the reaction: 1D-myo-inositol 1,3,4-trisphosphate + ATP = 1D-myo-inositol 1,3,4,5-tetrakisphosphate + ADP + H+. Sources: RHEA:13253